{
  "gene_symbol": "H2BC15",
  "term_label": "nucleus",
  "term_id": "GO:0005634",
  "gene_name": "Histone H2B type 1-N",
  "gene": "UniProtKB:Q99877"
}